{
  "gene_name": "Putative heat shock protein HSP 90-beta 4",
  "term_id": "GO:0032991",
  "gene": "UniProtKB:Q58FF6",
  "gene_symbol": "HSP90AB4P",
  "term_label": "protein-containing complex"
}